{
  "gene": "UniProtKB:O15304",
  "gene_symbol": "SIVA1",
  "gene_name": "Apoptosis regulatory protein Siva",
  "term_label": "extrinsic apoptotic signaling pathway",
  "term_id": "GO:0097191"
}